sporulation resulting in formation of a multicellular or syncytial spore [GO:0075283] (biological process) Also known as: multicellular or syncytial spore formation by sporulation Subtypes: asexual sporulation resulting in formation of a multicellular or syncytial spore [GO:0075284], sexual sporulation resulting in formation of a multicellular or syncytial spore [GO:0075285] Sources: GOC:pamgo_curators Relationships: is a type of sporulation [GO:0043934] Definition: The process whose specific outcome is the progression of a multicellular or syncytial spore via septations over time, from its initiation to the mature structure.